{
  "gene": "UniProtKB:O14893",
  "term_label": "Unknown molecular function",
  "gene_name": "Gem-associated protein 2",
  "term_id": "UNKNOWN:0001",
  "gene_symbol": "GEMIN2"
}